Roundabout signaling pathway involved in muscle cell chemotaxis toward tendon cell [GO:2001283] (biological process) Definition: Any Roundabout signaling pathway that is involved in the directed movement of a muscle cell towards a tendon cell in response to an external stimulus. References: PMID:19793885 Sources: GOC:bf, GOC:obol, GOC:sart Also known as: ROBO signaling pathway involved in muscle cell chemotaxis toward tendon cell, ROBO signaling pathway involved in muscle cell chemotaxis towards tendon cell, ROBO/SLIT signaling pathway involved in muscle cell chemotaxis toward tendon cell, ROBO/SLIT signaling pathway involved in muscle cell chemotaxis towards tendon cell, Roundabout signaling pathway involved in muscle cell chemotaxis towards tendon cell, Roundabout signalling pathway involved in muscle cell chemotaxis toward tendon cell, Roundabout signalling pathway involved in muscle cell chemotaxis towards tendon cell, ROBO signaling pathway involved in muscle cell attraction, ROBO/SLIT signaling pathway involved in muscle cell attraction, Roundabout signaling pathway involved in muscle cell attraction, Roundabout signalling pathway involved in muscle cell attraction Relationships: is a type of Roundabout signaling pathway [GO:0035385]; is part of muscle cell chemotaxis toward tendon cell [GO:0036061]